{
  "term_label": "endosome",
  "gene_name": "Sorting nexin-10",
  "gene": "UniProtKB:Q9Y5X0",
  "gene_symbol": "SNX10",
  "term_id": "GO:0005768"
}